{
  "term_id": "GO:0003743",
  "gene": "UniProtKB:B5ME19",
  "gene_symbol": "EIF3CL",
  "term_label": "translation initiation factor activity",
  "gene_name": "Eukaryotic translation initiation factor 3 subunit C-like protein"
}